{
  "gene_symbol": "SAMD10",
  "term_id": "UNKNOWN:0001",
  "term_label": "Unknown molecular function",
  "gene_name": "Sterile alpha motif domain-containing protein 10",
  "gene": "UniProtKB:Q9BYL1"
}